positive regulation of plant organ morphogenesis [GO:1905423] (biological process) Sources: GOC:TermGenie, GOC:tb, GO_REF:0000058 Definition: Any process that activates or increases the frequency, rate or extent of plant organ morphogenesis. Also known as: up regulation of plant organ morphogenesis, up-regulation of plant organ morphogenesis, upregulation of plant organ morphogenesis, activation of plant organ morphogenesis Relationships: is a type of positive regulation of developmental process [GO:0051094]; is_a positive regulation of multicellular organismal process [GO:0051240]; is a type of regulation of plant organ morphogenesis [GO:1905421]; positively regulates plant organ morphogenesis [GO:1905392]